{
  "term_id": "UNKNOWN:0003",
  "gene_symbol": "SLC20A2",
  "gene": "UniProtKB:Q08357",
  "term_label": "Unknown cellular component",
  "gene_name": "Sodium-dependent phosphate transporter 2"
}